DNA-methyltransferase activity [GO:0009008] (molecular function) Definition: Catalysis of the transfer of a methyl group to a DNA molecule. References: PMID:7862522 Sources: GOC:jl, ISBN:0198506732 Also known as: DNA methylase, DNA methyltransferase activity, DNA transmethylase activity, deoxyribonucleate methylase activity, deoxyribonucleate methyltransferase activity, deoxyribonucleic acid methylase activity, deoxyribonucleic acid methyltransferase activity, Type II DNA methylase, deoxyribonucleic acid modification methylase activity Relationships: is a type of methyltransferase activity [GO:0008168]; is_a catalytic activity, acting on DNA [GO:0140097] Subtypes: DNA (cytosine-5-)-methyltransferase activity [GO:0003886], site-specific DNA-methyltransferase (adenine-specific) activity [GO:0009007], site-specific DNA-methyltransferase (cytosine-N4-specific) activity [GO:0015667]